{
  "gene": "UniProtKB:O60688",
  "gene_symbol": "YPEL1",
  "gene_name": "Protein yippee-like 1",
  "term_id": "UNKNOWN:0003",
  "term_label": "Unknown cellular component"
}